O-fucosylpeptide 3-beta-glucosyltransferase activity [GO:0160265] (molecular function) References: PMID:16899492 Definition: Catalysis of the transfer of a alpha-D-glucose residue from UDP-alpha-D-glucose to the fucose residue of a fucosylated protein acceptor. Relationships: is a type of UDP-glucosyltransferase activity [GO:0035251]